{
  "gene_symbol": "FTSJ1",
  "gene_name": "Putative tRNA (cytidine(32)_guanosine(34)-2'-O)-methyltransferase",
  "gene": "UniProtKB:Q9UET6",
  "term_label": "tRNA methyltransferase activity",
  "term_id": "GO:0008175"
}